positive regulation of T cell costimulation [GO:2000525] (biological process) Also known as: positive regulation of T cell co-stimulation, positive regulation of T lymphocyte costimulation, positive regulation of T-cell co-stimulation, positive regulation of T-cell costimulation, positive regulation of T-lymphocyte costimulation Definition: Any process that activates or increases the frequency, rate or extent of T cell costimulation. Relationships: is a type of positive regulation of T cell activation [GO:0050870]; is a type of regulation of T cell costimulation [GO:2000523]; positively regulates GO:0031295 Sources: GOC:obol Subtypes: positive regulation of CD4-positive, alpha-beta T cell costimulation [GO:1900281]